{
  "gene": "UniProtKB:Q8NI08",
  "term_label": "response to oxidative stress",
  "gene_symbol": "NCOA7",
  "gene_name": "Nuclear receptor coactivator 7",
  "term_id": "GO:0006979"
}